{
  "gene_symbol": "IFNA17",
  "term_label": "cytokine activity",
  "term_id": "GO:0005125",
  "gene_name": "Interferon alpha-17",
  "gene": "UniProtKB:P01571"
}